{
  "gene_name": "Zinc finger protein 561",
  "gene_symbol": "ZNF561",
  "term_label": "nucleus",
  "term_id": "GO:0005634",
  "gene": "UniProtKB:Q8N587"
}